{
  "gene_symbol": "TMEM38A",
  "term_id": "GO:0016529",
  "term_label": "sarcoplasmic reticulum",
  "gene": "UniProtKB:Q9H6F2",
  "gene_name": "Trimeric intracellular cation channel type A"
}